{
  "gene_symbol": "CHRNB1",
  "term_label": "neuron projection",
  "gene_name": "Acetylcholine receptor subunit beta",
  "gene": "UniProtKB:P11230",
  "term_id": "GO:0043005"
}